{
  "term_label": "chromatin binding",
  "term_id": "GO:0003682",
  "gene_symbol": "MBD6",
  "gene_name": "Methyl-CpG-binding domain protein 6",
  "gene": "UniProtKB:Q96DN6"
}